{
  "gene_symbol": "TSEN54",
  "gene": "UniProtKB:Q7Z6J9",
  "term_label": "tRNA-intron endonuclease complex",
  "term_id": "GO:0000214",
  "gene_name": "tRNA-splicing endonuclease subunit Sen54"
}